{
  "term_id": "GO:0016485",
  "gene_name": "Cysteine protease ATG4C",
  "gene_symbol": "ATG4C",
  "gene": "UniProtKB:Q96DT6",
  "term_label": "protein processing"
}